negative regulation of small intestinal transit [GO:0120059] (biological process) Definition: Any process that decreases the frequency, rate or extent of any small intestinal transit process, the migration of ingested material along the length of the small intestine. Also known as: negative regulation of small bowel transit, negative regulation of small intestine transit References: PMID:15890336 Sources: GOC:sl Relationships: is a type of GO:0060457; is a type of regulation of small intestinal transit [GO:0120057]; negatively regulates small intestinal transit [GO:0120055]